{
  "gene_symbol": "HMG20B",
  "term_label": "Unknown molecular function",
  "gene_name": "SWI_SNF-related matrix-associated actin-dependent regulator of chromatin subfamily E member 1-related",
  "gene": "UniProtKB:Q9P0W2",
  "term_id": "UNKNOWN:0001"
}